regulation of antimicrobial peptide biosynthetic process [GO:0002805] (BP) Definition: Any process that modulates the frequency, rate, or extent of antimicrobial peptide biosynthesis. Subtypes: negative regulation of antimicrobial peptide biosynthetic process [GO:0002806], positive regulation of antimicrobial peptide biosynthetic process [GO:0002807], regulation of antibacterial peptide biosynthetic process [GO:0002808], regulation of antifungal peptide biosynthetic process [GO:0002810] Sources: GOC:add Relationships: is_a GO:0002784; RO_0002211 antimicrobial peptide biosynthetic process [GO:0002777]